{
  "term_id": "GO:0036064",
  "gene_name": "Centriole and centriolar satellite protein OFD1",
  "gene_symbol": "OFD1",
  "term_label": "ciliary basal body",
  "gene": "UniProtKB:O75665"
}